{
  "gene": "UniProtKB:Q7L1Q6",
  "gene_name": "eIF5-mimic protein 2",
  "term_id": "GO:0005737",
  "gene_symbol": "BZW1",
  "term_label": "cytoplasm"
}